{
  "gene_name": "Pro-FMRFamide-related neuropeptide FF",
  "term_id": "GO:0030425",
  "gene": "UniProtKB:O15130",
  "term_label": "dendrite",
  "gene_symbol": "NPFF"
}